negative regulation of feeding behavior [GO:2000252] (biological process) Definition: Any process that stops, prevents or reduces the frequency, rate or extent of feeding behavior. Subtypes: negative regulation of eating behavior [GO:1903999] Sources: GOC:obol Also known as: negative regulation of behavioral response to food, negative regulation of behavioural response to food, negative regulation of feeding behaviour, negative regulation of drinking, negative regulation of eating Relationships: is a type of negative regulation of behavior [GO:0048521]; is a type of regulation of feeding behavior [GO:0060259]; negatively regulates feeding behavior [GO:0007631]